gonadotropin-releasing hormone receptor activity [GO:0004968] (MF) Also known as: GnRH receptor activity, gonadotrophin-releasing hormone receptor activity Relationships: is a type of G protein-coupled receptor activity [GO:0004930]; is a type of protein-hormone receptor activity [GO:0016500]; BFO_0000050 cellular response to gonadotropin-releasing hormone [GO:0097211]; has part gonadotropin-releasing hormone binding [GO:0051448] Definition: Combining with gonadotropin-releasing hormone to initiate a change in cell activity. Gonadotropin-releasing hormone (GnRH) is a peptide hormone responsible for the release of follicle-stimulating hormone (FSH) and luteinizing hormone (LH) from the anterior pituitary. GnRH is synthesized and released by the hypothalamus. Sources: GOC:mah